protein de-ADP-ribosylation [GO:0051725] (BP) Definition: The process of removing one or more ADP-ribose residues from a protein. Relationships: is a type of protein modification process [GO:0036211] Sources: GOC:ai Subtypes: GO:0140290, peptidyl-glutamate ADP-deribosylation [GO:0140291] Also known as: poly(ADP-ribose) removal from protein, protein amino acid de-ADP-ribosylation, protein poly(ADP-ribose) catabolic process, protein poly(ADP-ribose) catabolism, protein poly(ADP-ribose) degradation, protein poly(ADP-ribose) hydrolysis, removal of ADP-ribose from protein